cell junction disassembly [GO:0150146] (biological process) Relationships: is a type of GO:0022411; is a type of cell junction organization [GO:0034330] References: PMID:25490267 Sources: GOC:aruk Subtypes: GO:0098883, GO:0120180, cell-cell junction disassembly [GO:0150147] Definition: The disaggregation of a cell junction into its constituent components.